{
  "gene_symbol": "GREB1L",
  "gene_name": "GREB1-like protein",
  "term_label": "Unknown cellular component",
  "gene": "UniProtKB:Q9C091",
  "term_id": "UNKNOWN:0003"
}